regulation of R7 cell differentiation [GO:0045676] (biological process) Sources: GOC:go_curators Definition: Any process that modulates the frequency, rate or extent of R7 differentiation. Subtypes: regulation of sevenless signaling pathway [GO:0045501], negative regulation of R7 cell differentiation [GO:0045677], GO:0045678 Relationships: is a type of regulation of compound eye photoreceptor cell differentiation [GO:0110116]; regulates GO:0045466